regulation of Frizzled Nuclear Import pathway [GO:0140710] (biological process) Relationships: is a type of regulation of non-canonical Wnt signaling pathway [GO:2000050]; RO_0002211 GO:0140709 Definition: Any process that modulates the frequency, rate or extent of a Frizzled Nuclear Import pathway. References: PMID:22510459, PMID:22579286 Subtypes: positive regulation of Frizzled Nuclear Import pathway [GO:0140711], negative regulation of Frizzled Nuclear Import pathway [GO:0140712] Also known as: regulation of FNI, regulation of Frizzled Nuclear Import Wnt Pathway